{
  "term_id": "UNKNOWN:0002",
  "gene": "UniProtKB:E5RG02",
  "term_label": "Unknown biological process",
  "gene_symbol": "PRSS46P",
  "gene_name": "Putative serine protease 46"
}